{
  "gene_name": "RUS family member 1",
  "gene": "UniProtKB:Q96GQ5",
  "term_label": "Unknown cellular component",
  "term_id": "UNKNOWN:0003",
  "gene_symbol": "RUSF1"
}